{
  "term_id": "UNKNOWN:0001",
  "term_label": "Unknown molecular function",
  "gene_symbol": "PRMT5",
  "gene": "UniProtKB:O14744",
  "gene_name": "Protein arginine N-methyltransferase 5"
}